focal adhesion [GO:0005925] (cellular component) Also known as: HAJ, connecting hemi-adherens junction, focal contact, hemi-adherens junction, adhesion plaque Relationships: is a type of GO:0030055 Definition: A cell-substrate junction that anchors the cell to the extracellular matrix and that forms a point of termination of actin filaments. In insects focal adhesion has also been referred to as hemi-adherens junction (HAJ). References: PMID:10419689, PMID:12191915, PMID:15246682, PMID:1643657, PMID:16805308, PMID:19197329, PMID:23033047, PMID:26923917, PMID:28796323, PMID:8314002 Sources: GOC:aruk, GOC:bc, ISBN:0124325653, ISBN:0815316208